{
  "gene_symbol": "TRHR",
  "gene_name": "Thyrotropin-releasing hormone receptor",
  "term_label": "Unknown cellular component",
  "term_id": "UNKNOWN:0003",
  "gene": "UniProtKB:P34981"
}